{
  "gene": "UniProtKB:Q8IXB3",
  "term_id": "GO:0032869",
  "term_label": "cellular response to insulin stimulus",
  "gene_symbol": "TRARG1",
  "gene_name": "Trafficking regulator of GLUT4 1"
}